{
  "term_id": "UNKNOWN:0001",
  "gene_symbol": "CELF2-AS1",
  "gene_name": "Putative uncharacterized protein CELF2-AS1",
  "term_label": "Unknown molecular function",
  "gene": "UniProtKB:Q8N7Q2"
}